{
  "term_label": "protein phosphatase regulator activity",
  "gene_name": "Protein phosphatase 1 regulatory subunit 15B",
  "gene": "UniProtKB:Q5SWA1",
  "gene_symbol": "PPP1R15B",
  "term_id": "GO:0019888"
}